{
  "gene_name": "Galectin-3",
  "term_id": "GO:0045806",
  "term_label": "negative regulation of endocytosis",
  "gene_symbol": "LGALS3",
  "gene": "UniProtKB:P17931"
}